{
  "gene_name": "Zinc finger and BTB domain-containing protein 16",
  "term_label": "DNA-binding transcription activator activity, RNA polymerase II-specific",
  "term_id": "GO:0001228",
  "gene": "UniProtKB:Q05516",
  "gene_symbol": "ZBTB16"
}